positive regulation of glycoprotein metabolic process [GO:1903020] (biological process) Definition: Any process that activates or increases the frequency, rate or extent of glycoprotein metabolic process. References: PMID:23544079 Sources: GOC:BHF, GOC:TermGenie, GOC:rl, GO_REF:0000058 Also known as: positive regulation of glycoprotein metabolism, up regulation of glycoprotein metabolic process, up regulation of glycoprotein metabolism, up-regulation of glycoprotein metabolic process, up-regulation of glycoprotein metabolism, upregulation of glycoprotein metabolic process, upregulation of glycoprotein metabolism, activation of glycoprotein metabolic process, activation of glycoprotein metabolism Note: human serum amyloid P component (SAP) P02743 inhibits viral neuraminidase, NA (exo-alpha-sialidase activity) and thus the metabolism of glycoproteins, demonstrated in Figure 4A PMID:23544079, (IDA), the negative regulation term would be applied to this protein Relationships: is_a GO:0051247; is a type of regulation of glycoprotein metabolic process [GO:1903018]; positively regulates glycoprotein metabolic process [GO:0009100] Subtypes: GO:0010560, positive regulation of elastin catabolic process [GO:0110015]